{
  "gene_name": "E3 ubiquitin-protein ligase TRIM21",
  "term_label": "innate immune response",
  "gene_symbol": "TRIM21",
  "gene": "UniProtKB:P19474",
  "term_id": "GO:0045087"
}